hydroxyacylglutathione hydrolase activity [GO:0004416] (molecular function) Also known as: S-(2-hydroxyacyl)glutathione hydrolase activity, S-2-hydroxylacylglutathione hydrolase activity, acetoacetylglutathione hydrolase activity, glyoxalase II activity Sources: RHEA:21864 Definition: Catalysis of the reaction: an S-(2-hydroxyacyl)glutathione + H2O = a 2-hydroxy carboxylate + glutathione + H+. Relationships: is a type of thiolester hydrolase activity [GO:0016790]